{
  "term_label": "RNA polymerase II transcription regulatory region sequence-specific DNA binding",
  "gene": "UniProtKB:Q7Z398",
  "gene_symbol": "ZNF550",
  "gene_name": "Zinc finger protein 550",
  "term_id": "GO:0000977"
}